secondary lysosome [GO:0005767] (cellular component) Relationships: is a type of lysosome [GO:0005764] Sources: GOC:jl, ISBN:0815316194 Subtypes: GO:0032010, autolysosome [GO:0044754] Definition: Vacuole formed by the fusion of a lysosome with an organelle (autosome) or with a primary phagosome.